{
  "term_label": "secretory granule",
  "gene_symbol": "PTPRN",
  "term_id": "GO:0030141",
  "gene_name": "Receptor-type tyrosine-protein phosphatase-like N",
  "gene": "UniProtKB:Q16849"
}